{
  "gene_symbol": "PSMC5",
  "term_id": "GO:0043161",
  "gene_name": "26S proteasome regulatory subunit 8",
  "gene": "UniProtKB:P62195",
  "term_label": "proteasome-mediated ubiquitin-dependent protein catabolic process"
}